{
  "gene_symbol": "ACAT2",
  "term_label": "Unknown cellular component",
  "gene_name": "Acetyl-CoA acetyltransferase, cytosolic",
  "gene": "UniProtKB:Q9BWD1",
  "term_id": "UNKNOWN:0003"
}